negative regulation of heart growth [GO:0061117] (biological process) Definition: Any process that decreases the rate or extent of heart growth. Heart growth is the increase in size or mass of the heart. Relationships: is a type of negative regulation of organ growth [GO:0046621]; is a type of GO:0060420; negatively regulates heart growth [GO:0060419] Subtypes: GO:0055022 Sources: GOC:dph, GOC:hjd